{
  "term_label": "regulation of actin nucleation",
  "term_id": "GO:0051125",
  "gene": "UniProtKB:Q12768",
  "gene_name": "WASH complex subunit 5",
  "gene_symbol": "WASHC5"
}